{
  "gene_symbol": "APOC2",
  "term_label": "high-density lipoprotein particle clearance",
  "gene_name": "Apolipoprotein C-II",
  "gene": "UniProtKB:P02655",
  "term_id": "GO:0034384"
}